{
  "term_label": "Unknown biological process",
  "gene_name": "TBC1 domain family member 15",
  "term_id": "UNKNOWN:0002",
  "gene_symbol": "TBC1D15",
  "gene": "UniProtKB:Q8TC07"
}